L-serine metabolic process [GO:0006563] (biological process) Relationships: is a type of GO:0170033; is a type of proteinogenic amino acid metabolic process [GO:0170039] Sources: GOC:ai, GOC:jsg Subtypes: cysteine biosynthetic process from serine [GO:0006535], L-serine biosynthetic process [GO:0006564], L-serine catabolic process [GO:0006565], glycine biosynthetic process from serine [GO:0019264] Definition: The chemical reactions and pathways involving L-serine, the L-enantiomer of serine, i.e. (2S)-2-amino-3-hydroxypropanoic acid. Also known as: L-serine metabolism